{
  "gene_symbol": "MECP2",
  "gene": "UniProtKB:P51608",
  "term_label": "chromatin binding",
  "term_id": "GO:0003682",
  "gene_name": "Methyl-CpG-binding protein 2"
}